hypoxia-inducible factor-1alpha signaling pathway [GO:0097411] (biological process) Relationships: is a type of intracellular signal transduction [GO:0035556]; is part of cellular response to hypoxia [GO:0071456] Regulation: regulated by regulation of hypoxia-inducible factor-1alpha signaling pathway [GO:1902071]; negatively regulated by negative regulation of hypoxia-inducible factor-1alpha signaling pathway [GO:1902072]; RO_0002213 by positive regulation of hypoxia-inducible factor-1alpha signaling pathway [GO:1902073] Also known as: HIF1alpha pathway, hypoxia-inducible factor signaling, hypoxia-inducible factor-1alpha signalling pathway Definition: The series of molecular signals mediated by hypoxia-inducible factor (HIF1) in response to lowered oxygen levels (hypoxia). Under hypoxic conditions, the oxygen-sensitive alpha-subunit of hypoxia-inducible factor (HIF)-1 dimerizes with a HIF1-beta subunit (also called ARNT or aryl-hydrocarbon-receptor nuclear translocator), translocates to the nucleus and activates transcription of genes whose products participate in responding to hypoxia. References: PMID:16887934, PMID:26579469 Sources: GOC:bf, GOC:jc